{
  "gene": "UniProtKB:Q8IWB6",
  "term_id": "GO:0045171",
  "gene_symbol": "TEX14",
  "term_label": "intercellular bridge",
  "gene_name": "Inactive serine_threonine-protein kinase TEX14"
}